thigmotropism [GO:0009652] (biological process) Relationships: is a type of tropism [GO:0009606]; is a type of response to mechanical stimulus [GO:0009612] Definition: The movement of an organism, or part of an organism, such as leaves or tendrils, in response to a touch stimulus, usually toward or away from it. References: PMID:16153165 Sources: GOC:jl